Schwann cell migration [GO:0036135] (biological process) References: PMID:20335460 Sources: CL:0002573 Regulation: regulated by regulation of Schwann cell migration [GO:1900147]; negatively regulated by negative regulation of Schwann cell migration [GO:1900148]; positively regulated by positive regulation of Schwann cell migration [GO:1900149] Subtypes: Schwann cell chemotaxis [GO:1990751] Relationships: is a type of glial cell migration [GO:0008347] Definition: The orderly movement of a Schwann cell from one site to another. A Schwann cell is a glial cell that ensheathes axons of neuron in the peripheral nervous system and is necessary for their maintenance and function.